regulation of alcohol biosynthetic process [GO:1902930] (biological process) Also known as: regulation of solventogenesis, regulation of alcohol anabolism, regulation of alcohol biosynthesis, regulation of alcohol formation, regulation of alcohol synthesis Relationships: is a type of regulation of biosynthetic process [GO:0009889]; is a type of regulation of small molecule metabolic process [GO:0062012]; regulates alcohol biosynthetic process [GO:0046165] Definition: Any process that modulates the frequency, rate or extent of alcohol biosynthetic process. Subtypes: regulation of abscisic acid biosynthetic process [GO:0010115], regulation of inositol phosphate biosynthetic process [GO:0010919], GO:0032347, regulation of ergosterol biosynthetic process [GO:0032443], regulation of cholesterol biosynthetic process [GO:0045540], GO:0070623, regulation of inositol biosynthetic process [GO:1900088], GO:1900394, regulation of butyryl-CoA catabolic process to butanol [GO:1900497], GO:1900637, regulation of neosartoricin biosynthetic process [GO:1902053], GO:1902931, positive regulation of alcohol biosynthetic process [GO:1902932], regulation of phytol biosynthetic process [GO:1904963], GO:2000064 References: PMID:23332010 Sources: GOC:TermGenie, GOC:mengo_curators, GO_REF:0000058